{
  "term_id": "GO:0004984",
  "gene": "UniProtKB:Q15615",
  "term_label": "olfactory receptor activity",
  "gene_symbol": "OR4D1",
  "gene_name": "Olfactory receptor 4D1"
}